{
  "gene_name": "Regulator of G-protein signaling 4",
  "term_label": "GTPase activator activity",
  "term_id": "GO:0005096",
  "gene_symbol": "RGS4",
  "gene": "UniProtKB:P49798"
}